{
  "term_id": "GO:0070740",
  "gene_name": "Tubulin polyglutamylase TTLL6",
  "gene_symbol": "TTLL6",
  "gene": "UniProtKB:Q8N841",
  "term_label": "tubulin-glutamic acid ligase activity"
}